nucleobase metabolic process [GO:0009112] (biological process) Definition: The chemical reactions and pathways involving a nucleobase, a nitrogenous base that is a constituent of a nucleic acid, e.g. the purines: adenine, guanine, hypoxanthine, xanthine and the pyrimidines: cytosine, uracil, thymine. Relationships: is a type of nucleobase-containing small molecule metabolic process [GO:0055086] Also known as: nucleobase metabolism Subtypes: purine nucleobase metabolic process [GO:0006144], pyrimidine nucleobase metabolic process [GO:0006206], nucleobase biosynthetic process [GO:0046112], nucleobase catabolic process [GO:0046113] Sources: GOC:ma